proteolysis associated with antigen processing and presentation [GO:0002496] (biological process) Regulation: regulated by regulation of proteolysis associated with antigen processing and presentation [GO:0002628]; negatively regulated by negative regulation of proteolysis associated with antigen processing and presentation [GO:0002629]; positively regulated by positive regulation of proteolysis associated with antigen processing and presentation [GO:0002630] Relationships: is a type of GO:0051603; is part of antigen processing and presentation of peptide antigen [GO:0048002] Subtypes: proteolysis by cytosolic proteases associated with antigen processing and presentation [GO:0002203], proteasomal proteolysis associated with antigen processing and presentation [GO:0002497], proteolysis within endoplasmic reticulum associated with antigen processing and presentation [GO:0002498], proteolysis within endosome associated with antigen processing and presentation [GO:0002499], proteolysis within lysosome associated with antigen processing and presentation [GO:0002500] Definition: The hydrolysis of a peptide bond or bonds within a protein contributing to antigen processing and presentation. References: PMID:15224092, PMID:15771591 Sources: GOC:add, ISBN:0781735149